{
  "term_id": "GO:0006357",
  "gene_symbol": "MT-RNR1",
  "gene_name": "Mitochondrial-derived peptide MOTS-c",
  "term_label": "regulation of transcription by RNA polymerase II",
  "gene": "UniProtKB:A0A0C5B5G6"
}